quiescent center organization [GO:1904961] (biological process) References: PMID:21233333 Sources: GOC:TermGenie, GO_REF:0000084 Also known as: quiescent center structural organization Definition: The process that contributes to the act of creating the structural organization of the quiescent center. This process pertains to the physical shaping of a rudimentary structure. Relationships: is a type of anatomical structure arrangement [GO:0048532]